{
  "term_id": "UNKNOWN:0001",
  "gene_symbol": "UCMA",
  "gene": "UniProtKB:Q8WVF2",
  "term_label": "Unknown molecular function",
  "gene_name": "Unique cartilage matrix-associated protein"
}